{
  "term_id": "GO:0005891",
  "gene": "UniProtKB:Q9P0X4",
  "term_label": "voltage-gated calcium channel complex",
  "gene_symbol": "CACNA1I",
  "gene_name": "Voltage-dependent T-type calcium channel subunit alpha-1I"
}